{
  "gene_name": "CCR4-NOT transcription complex subunit 8",
  "gene": "UniProtKB:Q9UFF9",
  "gene_symbol": "CNOT8",
  "term_id": "GO:0004535",
  "term_label": "poly(A)-specific ribonuclease activity"
}